{
  "term_id": "UNKNOWN:0003",
  "term_label": "Unknown cellular component",
  "gene": "UniProtKB:Q9P1Z2",
  "gene_symbol": "CALCOCO1",
  "gene_name": "Calcium-binding and coiled-coil domain-containing protein 1"
}